{
  "term_label": "histone H3K4 monomethyltransferase activity",
  "gene_name": "Histone-lysine N-methyltransferase 2D",
  "term_id": "GO:0140945",
  "gene_symbol": "KMT2D",
  "gene": "UniProtKB:O14686"
}